{
  "gene_symbol": "TIMM17A",
  "term_label": "protein transmembrane transporter activity",
  "gene_name": "Mitochondrial import inner membrane translocase subunit Tim17-A",
  "gene": "UniProtKB:Q99595",
  "term_id": "GO:0008320"
}